detection of calcium ion [GO:0005513] (biological process) Also known as: Ca2+ ion detection, calcium ion detection, calcium ion sensing, detection of Ca2+ ion Sources: GOC:pg Relationships: is a type of detection of chemical stimulus [GO:0009593]; is a type of response to calcium ion [GO:0051592] Definition: The series of events in which a calcium ion stimulus is received by a cell and converted into a molecular signal.